'de novo' cotranslational protein folding [GO:0051083] (biological process) Definition: The process of assisting in the correct noncovalent assembly of the ribosome-bound nascent chains of a multidomain protein whilst other parts of the protein are still being translated. Sources: GOC:rb Also known as: 'de novo' co-translational protein folding, multidomain protein assembly, nascent polypeptide association Relationships: is a type of 'de novo' protein folding [GO:0006458]